{
  "gene": "UniProtKB:O95630",
  "term_id": "GO:0046580",
  "gene_name": "STAM-binding protein",
  "term_label": "negative regulation of Ras protein signal transduction",
  "gene_symbol": "STAMBP"
}